{
  "term_id": "UNKNOWN:0001",
  "gene_symbol": "AADACL3",
  "gene": "UniProtKB:Q5VUY0",
  "term_label": "Unknown molecular function",
  "gene_name": "Arylacetamide deacetylase-like 3"
}